{
  "gene_symbol": "GRIPAP1",
  "gene": "UniProtKB:Q4V328",
  "term_label": "glutamatergic synapse",
  "term_id": "GO:0098978",
  "gene_name": "GRIP1-associated protein 1"
}